bacterial-type flagellum rotor complex [GO:0120107] (cellular component) Definition: The rotor complex of the bacterial-type flagellum consists of a membrane-anchored ring and the motor switch complex, which participates in the conversion of proton/Na+ energy into the mechanical work of rotation and controls the direction of flagellar rotation. Relationships: is a type of cellular anatomical structure [GO:0110165]; is part of GO:0120100 References: PMID:10572114, PMID:12624192, PMID:25251856 Sources: GOC:cilia